{
  "gene_name": "UDP-GalNAc:beta-1,3-N-acetylgalactosaminyltransferase 2",
  "term_id": "GO:0008194",
  "gene_symbol": "B3GALNT2",
  "term_label": "UDP-glycosyltransferase activity",
  "gene": "UniProtKB:Q8NCR0"
}